{
  "term_label": "positive regulation of JNK cascade",
  "term_id": "GO:0046330",
  "gene_symbol": "EDA2R",
  "gene": "UniProtKB:Q9HAV5",
  "gene_name": "Tumor necrosis factor receptor superfamily member 27"
}